{
  "gene_symbol": "GRIK5",
  "term_label": "kainate selective glutamate receptor activity",
  "gene_name": "Glutamate receptor ionotropic, kainate 5",
  "term_id": "GO:0015277",
  "gene": "UniProtKB:Q16478"
}